{
  "term_id": "GO:0005768",
  "gene_name": "Phosphatidylinositol 4-kinase type 2-alpha",
  "gene_symbol": "PI4K2A",
  "term_label": "endosome",
  "gene": "UniProtKB:Q9BTU6"
}